chlorophyll catabolite transmembrane transporter activity [GO:0010290] (molecular function) Relationships: is a type of transmembrane transporter activity [GO:0022857] References: PMID:9681016 Definition: Enables the directed movement of chlorophyll catabolites such as non-fluorescent chlorophyll catabolites (NCCs), from one side of a membrane to the other.